{
  "term_label": "cell differentiation",
  "gene_name": "Forkhead box protein D3",
  "gene_symbol": "FOXD3",
  "term_id": "GO:0030154",
  "gene": "UniProtKB:Q9UJU5"
}